{
  "gene_name": "Geranylgeranyl transferase type-2 subunit alpha",
  "term_label": "Rab-protein geranylgeranyltransferase complex",
  "term_id": "GO:0005968",
  "gene_symbol": "RABGGTA",
  "gene": "UniProtKB:Q92696"
}